{
  "gene_symbol": "OR8G3",
  "gene": "UniProtKB:P0DMU2",
  "term_id": "GO:0007186",
  "gene_name": "Putative olfactory receptor 8G3 pseudogene",
  "term_label": "G protein-coupled receptor signaling pathway"
}